{
  "term_id": "GO:0003723",
  "gene": "UniProtKB:Q14296",
  "term_label": "RNA binding",
  "gene_symbol": "FASTK",
  "gene_name": "Fas-activated serine_threonine kinase"
}